nucleus leading edge [GO:0110092] (cellular component) Relationships: is a type of cellular anatomical structure [GO:0110165]; is part of nucleus [GO:0005634] References: PMID:15030757, PMID:24335254 Sources: GOC:al, GOC:mah, GOC:vw Definition: The area of a motile nucleus closest to the direction of movement. Also known as: horsetail nucleus leading edge